{
  "gene_symbol": "TNKS2",
  "gene_name": "Poly [ADP-ribose] polymerase tankyrase-2",
  "gene": "UniProtKB:Q9H2K2",
  "term_label": "cytoplasm",
  "term_id": "GO:0005737"
}